{
  "gene": "UniProtKB:Q8IY42",
  "term_id": "UNKNOWN:0002",
  "gene_name": "Uncharacterized protein C4orf19",
  "gene_symbol": "C4orf19",
  "term_label": "Unknown biological process"
}